{
  "term_label": "transmembrane signaling receptor activity",
  "term_id": "GO:0004888",
  "gene": "UniProtKB:Q6UXG3",
  "gene_name": "CMRF35-like molecule 9",
  "gene_symbol": "CD300LG"
}